{
  "gene": "UniProtKB:P30048",
  "term_id": "GO:0006979",
  "gene_symbol": "PRDX3",
  "term_label": "response to oxidative stress",
  "gene_name": "Thioredoxin-dependent peroxide reductase, mitochondrial"
}